regulation of cell adhesion [GO:0030155] (biological process) Relationships: is a type of regulation of cellular process [GO:0050794]; regulates cell adhesion [GO:0007155] Definition: Any process that modulates the frequency, rate or extent of attachment of a cell to another cell or to the extracellular matrix. Sources: GOC:mah Subtypes: regulation of cell adhesion involved in intussusceptive angiogenesis [GO:0002045], GO:0003436, negative regulation of cell adhesion [GO:0007162], GO:0010810, regulation of cell-cell adhesion [GO:0022407], GO:0033628, positive regulation of cell adhesion [GO:0045785], GO:0061344, regulation of cell adhesion involved in sprouting angiogenesis [GO:0106088] Also known as: cell adhesion receptor regulator activity